pentalenolactone biosynthetic process [GO:1901780] (biological process) Definition: The chemical reactions and pathways resulting in the formation of pentalenolactone. References: PMID:17178094 Sources: GOC:TermGenie, GOC:yaf, MetaCyc:PWY-6915, UniPathway:UPA00974 Also known as: pentalenolactone anabolism, pentalenolactone biosynthesis, pentalenolactone formation, pentalenolactone synthesis Relationships: is a type of sesquiterpenoid biosynthetic process [GO:0016106]; is a type of monocarboxylic acid biosynthetic process [GO:0072330]; is a type of epoxide metabolic process [GO:0097176]; is a type of lactone biosynthetic process [GO:1901336]; is a type of GO:1901503